{
  "gene_symbol": "KNDC1",
  "term_id": "GO:0048814",
  "gene": "UniProtKB:Q76NI1",
  "term_label": "regulation of dendrite morphogenesis",
  "gene_name": "Kinase non-catalytic C-lobe domain-containing protein 1"
}